{
  "term_label": "penetration of zona pellucida",
  "gene_name": "Nuclear transition protein 2",
  "gene": "UniProtKB:Q05952",
  "term_id": "GO:0007341",
  "gene_symbol": "TNP2"
}